{
  "term_id": "GO:0050852",
  "gene_name": "T-cell-specific surface glycoprotein CD28",
  "term_label": "T cell receptor signaling pathway",
  "gene_symbol": "CD28",
  "gene": "UniProtKB:P10747"
}